{
  "term_id": "GO:0035330",
  "gene_name": "Merlin",
  "gene_symbol": "NF2",
  "gene": "UniProtKB:P35240",
  "term_label": "regulation of hippo signaling"
}